negative regulation of eye pigmentation [GO:0048074] (biological process) Sources: GOC:jid Also known as: down regulation of eye pigmentation, down-regulation of eye pigmentation, downregulation of eye pigmentation, inhibition of eye pigmentation Definition: Any process that stops, prevents, or reduces the frequency, rate or extent of establishment of a pattern of pigment in the eye of an organism. Subtypes: negative regulation of compound eye pigmentation [GO:0048077] Relationships: is a type of GO:0048073; is a type of negative regulation of developmental pigmentation [GO:0048086]; negatively regulates GO:0048069